{
  "gene_symbol": "A0A8I5QKY2",
  "term_label": "Unknown cellular component",
  "term_id": "UNKNOWN:0003",
  "gene_name": "Uncharacterized protein",
  "gene": "UniProtKB:A0A8I5QKY2"
}